1,3-beta-D-glucan synthase activity [GO:0003843] (molecular function) Definition: Catalysis of the reaction: UDP-glucose + [(1->3)-beta-D-glucosyl](n) = UDP + [(1->3)-beta-D-glucosyl](n+1). Sources: EC:2.4.1.34 Also known as: beta-1,3-glucan synthase activity, callose synthase activity, (1,3)-beta-glucan (callose) synthase activity, 1,3-beta-D-glucan synthetase activity, 1,3-beta-D-glucan-UDP glucosyltransferase activity, 1,3-beta-glucan synthase activity, 1,3-beta-glucan-uridine diphosphoglucosyltransferase activity, GS-II, UDP-glucose-1,3-beta-D-glucan glucosyltransferase activity, UDP-glucose-1,3-beta-glucan glucosyltransferase activity, UDP-glucose-beta-glucan glucosyltransferase activity, UDP-glucose:(1,3)beta-glucan synthase activity, UDP-glucose:1,3-beta-D-glucan 3-beta-D-glucosyltransferase activity, UDPglucose-1,3-beta-D-glucan glucosyltransferase activity, UDPglucose:1,3-beta-D-glucan 3-beta-D-glucosyltransferase activity, beta-1,3-glucan synthetase activity, callose synthetase activity, paramylon synthetase, uridine diphosphoglucose-1,3-beta-glucan glucosyltransferase activity Relationships: is a type of UDP-glucosyltransferase activity [GO:0035251] Subtypes: branched 1,3-beta-D-glucan synthase activity [GO:0140752], GO:0140753